{
  "term_id": "UNKNOWN:0001",
  "gene": "UniProtKB:Q9Y3E0",
  "term_label": "Unknown molecular function",
  "gene_name": "Vesicle transport protein GOT1B",
  "gene_symbol": "GOLT1B"
}